(R)-benzylsuccinyl-CoA dehydrogenase activity [GO:0033734] (molecular function) Also known as: (R)-benzylsuccinyl-CoA:(acceptor) oxidoreductase activity, (R)-benzylsuccinyl-CoA:acceptor oxidoreductase activity, BbsG Relationships: is a type of oxidoreductase activity, acting on the CH-CH group of donors, with a flavin as acceptor [GO:0052890] Sources: EC:1.3.8.3 Definition: Catalysis of the reaction: (R)-2-benzylsuccinyl-CoA + 2 electron-transferring flavoprotein = (E)-2-benzylidenesuccinyl-CoA + 2 reduced electron-transferring flavoprotein.